interferon regulatory factor complex [GO:0097071] (CC) Relationships: is a type of protein-containing complex [GO:0032991] Subtypes: interferon regulatory factor 3 complex [GO:0097072], interferon regulatory factor 5 complex [GO:0097073], GO:0097074, interferon regulatory factor 3-interferon regulatory factor 7 complex [GO:0097075], GO:0097085 Also known as: IRF complex References: PMID:20043992 Sources: GOC:cna Definition: A protein complex that consists of two interferon regulatory proteins (IRFs); may be homodimeric or heterodimeric. The activation of a latent closed conformation of IRF in the cytoplasm is triggered by phosphorylation of Ser/Thr residues in a C-terminal region. Phosphorylation stimulates the C-terminal autoinhibitory domain to attain a highly extended conformation triggering dimerization through extensive contacts to a second subunit.